{
  "term_label": "defense response to bacterium",
  "gene_symbol": "DEFB110",
  "gene_name": "Beta-defensin 110",
  "gene": "UniProtKB:Q30KQ9",
  "term_id": "GO:0042742"
}